response to type III interferon [GO:0034342] (biological process) Relationships: is a type of GO:0034097; BFO_0000050 innate immune response [GO:0045087] Subtypes: cellular response to type III interferon [GO:0071358] Also known as: response to type III IFN, response to interferon-lambda References: PMID:15546383, PMID:16734557 Sources: GOC:add, ISBN:0126896631 Definition: Any process that results in a change in state or activity of a cell or an organism (in terms of movement, secretion, enzyme production, gene expression, etc.) as a result of a type III interferon stimulus. Interferon lambda is the only member of the type III interferon found so far.